{
  "gene_name": "Claudin-3",
  "gene_symbol": "CLDN3",
  "gene": "UniProtKB:O15551",
  "term_id": "GO:0070830",
  "term_label": "bicellular tight junction assembly"
}